{
  "gene": "UniProtKB:O14599",
  "gene_name": "Testis-specific basic protein Y 2",
  "gene_symbol": "BPY2",
  "term_id": "GO:0007283",
  "term_label": "spermatogenesis"
}